3-cyanoalanine hydratase activity [GO:0047558] (molecular function) Also known as: L-asparagine hydro-lyase (3-cyanoalanine-forming), L-asparagine hydro-lyase activity, beta-CNA nitrilase activity, beta-CNAla hydrolase activity, beta-cyanoalanine hydratase activity, beta-cyanoalanine hydrolase activity Definition: Catalysis of the reaction: L-asparagine = 3-cyano-L-alanine + H2O + H+. Relationships: is a type of hydro-lyase activity [GO:0016836] Sources: EC:4.2.1.65, RHEA:15385